myosin binding [GO:0017022] (molecular function) Also known as: myosin phosphatase myosin binding Sources: GOC:mah Relationships: is a type of cytoskeletal protein binding [GO:0008092] Definition: Binding to a myosin; myosins are any of a superfamily of molecular motor proteins that bind to actin and use the energy of ATP hydrolysis to generate force and movement along actin filaments. Subtypes: myosin I binding [GO:0017024], myosin III binding [GO:0031473], myosin V binding [GO:0031489], myosin light chain binding [GO:0032027], myosin heavy chain binding [GO:0032036], myosin II binding [GO:0045159], myosin VI binding [GO:0070853]